{
  "term_id": "GO:0000981",
  "gene": "UniProtKB:Q8N9K5",
  "gene_symbol": "ZNF565",
  "gene_name": "Zinc finger protein 565",
  "term_label": "DNA-binding transcription factor activity, RNA polymerase II-specific"
}